{
  "term_id": "GO:0000978",
  "gene_name": "Zinc finger protein 644",
  "term_label": "RNA polymerase II cis-regulatory region sequence-specific DNA binding",
  "gene": "UniProtKB:Q9H582",
  "gene_symbol": "ZNF644"
}